phospholipid:diacylglycerol acyltransferase activity [GO:0046027] (molecular function) Definition: Catalysis of the reaction: a glycerophospholipid + a 1,2-diacyl-sn-glycerol = a monoacylglycerophospholipid + a triacyl-sn-glycerol. Sources: RHEA:14057 Also known as: PDAT activity, phospholipid:1,2-diacyl-sn-glycerol O-acyltransferase activity Relationships: is a type of GO:0016747